{
  "gene_name": "CCN family member 1",
  "term_label": "positive regulation of cell migration",
  "gene_symbol": "CCN1",
  "gene": "UniProtKB:O00622",
  "term_id": "GO:0030335"
}